centriole scaffold activity [GO:0140180] (molecular function) References: PMID:29784964, PMID:32956907, PMID:34702818 Definition: The binding activity of a protein that contributes to the stable formation of a centriole by forming persistent structures, or templates, upon which other centriolar proteins assemble. Relationships: is a type of protein-macromolecule adaptor activity [GO:0030674]